{
  "term_label": "plasma membrane",
  "gene": "UniProtKB:Q14957",
  "gene_name": "Glutamate receptor ionotropic, NMDA 2C",
  "gene_symbol": "GRIN2C",
  "term_id": "GO:0005886"
}